{
  "gene": "UniProtKB:Q9NR31",
  "gene_symbol": "SAR1A",
  "term_label": "COPII vesicle coat",
  "term_id": "GO:0030127",
  "gene_name": "GTP-binding protein SAR1a"
}